D-alanine-D-serine ligase activity [GO:0160222] (molecular function) Relationships: is a type of GO:0016881 Definition: Catalysis of the reaction: ATP + D-alanine + D-serine = ADP + D-alanyl-D-serine + H+ + phosphate. Sources: EC:6.3.2.35, RHEA:27706